xylitol transmembrane transport [GO:1902341] (biological process) Relationships: is a type of polyol transmembrane transport [GO:0015791]; is a type of GO:0034219 Definition: The directed movement of a xylitol across a membrane. Xylitol is a polyalcohol (pentane-1,2,3,4,5-pentol), produced by hydrogenation of xylose. Also known as: xylitol transport References: PMID:23475614 Sources: GOC:TermGenie